cellulose microfibril organization [GO:0010215] (biological process) Relationships: is a type of GO:0030198; is part of plant-type cell wall assembly [GO:0071668] Also known as: cellulose microfibril organisation Definition: A process that is carried out at the cellular level which results in the assembly, arrangement of constituent parts, or disassembly of a cellulose microfibril, any of the cellulose structures laid down in orthogonal layers in a plant cell wall. References: PMID:12468730 Sources: GOC:mah